cis-zeatin biosynthetic process [GO:0033465] (biological process) Definition: The chemical reactions and pathways resulting in the formation of cis-zeatin, (2Z)-2-methyl-4-(9H-purin-6-ylamino)but-2-en-1-ol. Sources: GOC:mah Also known as: cis-zeatin anabolism, cis-zeatin biosynthesis, cis-zeatin formation, cis-zeatin synthesis Relationships: is a type of zeatin biosynthetic process [GO:0033398]